negative regulation of response to alcohol [GO:1901420] (BP) Definition: Any process that stops, prevents or reduces the frequency, rate or extent of response to alcohol. Relationships: is a type of GO:0048585; is a type of regulation of response to alcohol [GO:1901419]; negatively regulates response to alcohol [GO:0097305] Also known as: down regulation of response to alcohol, down-regulation of response to alcohol, downregulation of response to alcohol, inhibition of response to alcohol Sources: GOC:TermGenie, GOC:mengo_curators Subtypes: negative regulation of response to ethanol [GO:1901417], negative regulation of response to propan-1-ol [GO:1901446], negative regulation of response to butan-1-ol [GO:1901449], GO:1905958